{
  "term_id": "GO:0030576",
  "gene_symbol": "USPL1",
  "gene": "UniProtKB:Q5W0Q7",
  "term_label": "Cajal body organization",
  "gene_name": "SUMO-specific isopeptidase USPL1"
}